{
  "gene": "UniProtKB:Q15906",
  "term_label": "Swr1 complex",
  "gene_symbol": "VPS72",
  "gene_name": "Vacuolar protein sorting-associated protein 72 homolog",
  "term_id": "GO:0000812"
}